negative regulation of catabolic process [GO:0009895] (biological process) Also known as: down regulation of catabolic process, down-regulation of catabolic process, downregulation of catabolic process, negative regulation of breakdown, negative regulation of catabolism, negative regulation of degradation, inhibition of catabolic process Relationships: is a type of negative regulation of metabolic process [GO:0009892]; is a type of GO:0009894; negatively regulates catabolic process [GO:0009056] Subtypes: negative regulation of autophagy [GO:0010507], negative regulation of collagen catabolic process [GO:0010711], negative regulation of nucleotide catabolic process [GO:0030812], negative regulation of amine catabolic process [GO:0033242], GO:0033248, negative regulation of amide catabolic process [GO:0034252], negative regulation of protein catabolic process [GO:0042177], negative regulation of acetate catabolic process [GO:0045753], negative regulation of glycogen catabolic process [GO:0045818], negative regulation of lipid catabolic process [GO:0050995], negative regulation of anthocyanin catabolic process [GO:1900001], GO:1900283, negative regulation of coenzyme F420-dependent bicyclic nitroimidazole catabolic process [GO:1900289], negative regulation of alcohol catabolic process [GO:1900420], negative regulation of xylose catabolic process to ethanol [GO:1900516], negative regulation of tetrapyrrole catabolic process [GO:1901405], negative regulation of toluene catabolic process [GO:1901435], negative regulation of ferulate catabolic process [GO:1901467], negative regulation of syringal lignin catabolic process [GO:1901470], negative regulation of gamma-aminobutyric acid catabolic process [GO:1901716], GO:1902369, negative regulation of ornithine catabolic process [GO:1903267], GO:1903625, negative regulation of glucose catabolic process to lactate via pyruvate [GO:1904024], negative regulation of ubiquitin-dependent protein catabolic process [GO:2000059], negative regulation of hydrogen peroxide catabolic process [GO:2000296], negative regulation of receptor catabolic process [GO:2000645], negative regulation of starch catabolic process [GO:2000882], negative regulation of glucomannan catabolic process [GO:2000907], negative regulation of galactoglucomannan catabolic process [GO:2000913], GO:2000928, negative regulation of cellotriose catabolic process [GO:2000937], negative regulation of cyclodextrin catabolic process [GO:2000958], negative regulation of cellooligosaccharide catabolic process [GO:2000964], GO:2000967, negative regulation of hemicellulose catabolic process [GO:2000989], negative regulation of galactomannan catabolic process [GO:2000992], negative regulation of cellulose catabolic process [GO:2000998], negative regulation of pectin catabolic process [GO:2001004], negative regulation of glycolytic fermentation to ethanol [GO:2001155], GO:2001157 Definition: Any process that stops, prevents, or reduces the frequency, rate or extent of the chemical reactions and pathways resulting in the breakdown of substances. Sources: GOC:go_curators